pyrimidine nucleoside triphosphate catabolic process [GO:0009149] (biological process) Also known as: pyrimidine nucleoside triphosphate breakdown, pyrimidine nucleoside triphosphate catabolism, pyrimidine nucleoside triphosphate degradation Definition: The chemical reactions and pathways resulting in the breakdown of pyrimidine nucleoside triphosphate, a compound consisting of a pyrimidine base linked to a ribose or deoxyribose sugar esterified with triphosphate on the sugar. Relationships: is a type of GO:0009143; is a type of pyrimidine nucleoside triphosphate metabolic process [GO:0009147] Subtypes: pyrimidine ribonucleoside triphosphate catabolic process [GO:0009210], GO:0009213 Sources: GOC:go_curators, ISBN:0198506732